{
  "gene_symbol": "RPLP1",
  "term_id": "GO:0043021",
  "gene_name": "Large ribosomal subunit protein P1",
  "gene": "UniProtKB:P05386",
  "term_label": "ribonucleoprotein complex binding"
}